{
  "gene": "UniProtKB:Q3MIR4",
  "gene_symbol": "TMEM30B",
  "term_id": "GO:0045332",
  "gene_name": "Cell cycle control protein 50B",
  "term_label": "phospholipid translocation"
}